{
  "gene_name": "Phospholipase A-2-activating protein",
  "gene_symbol": "PLAA",
  "term_id": "GO:0005634",
  "term_label": "nucleus",
  "gene": "UniProtKB:Q9Y263"
}